{
  "gene": "UniProtKB:Q9NP50",
  "gene_name": "SIN3-HDAC complex-associated factor",
  "term_label": "negative regulation of cell migration",
  "gene_symbol": "SINHCAF",
  "term_id": "GO:0030336"
}